formation of haustorium for nutrient acquisition [GO:0052094] (biological process) Also known as: formation by organism of haustoria for nutrient acquisition from host, formation by organism of haustorium for nutrient acquisition from host, formation by symbiont of haustorium for nutrient acquisition from host Sources: GOC:mtg_pamgo_17jul06 Relationships: is a type of GO:0052093 Definition: The assembly of a haustorium, a projection from a symbiotic cell or tissue that penetrates the host's tissues for the purpose of obtaining nutrients. The host is defined as the larger of the organisms involved in a symbiotic interaction. Regulation: regulated by regulation of formation by symbiont of haustorium for nutrient acquisition from host [GO:0075045]; positively regulated by positive regulation of formation by symbiont of haustorium for nutrient acquisition from host [GO:0075046]; negatively regulated by GO:0075047